{
  "term_id": "GO:0005829",
  "gene_name": "Ubiquitin carboxyl-terminal hydrolase 17-like protein 5",
  "term_label": "cytosol",
  "gene_symbol": "USP17L5",
  "gene": "UniProtKB:A8MUK1"
}